{
  "gene_name": "SWI_SNF complex subunit SMARCC1",
  "term_id": "GO:0071564",
  "gene_symbol": "SMARCC1",
  "term_label": "npBAF complex",
  "gene": "UniProtKB:Q92922"
}